{
  "term_label": "regulation of DNA-templated transcription",
  "gene": "UniProtKB:Q9NR22",
  "gene_symbol": "PRMT8",
  "gene_name": "Protein arginine N-methyltransferase 8",
  "term_id": "GO:0006355"
}